{
  "gene": "UniProtKB:Q6IF00",
  "gene_symbol": "OR2T2",
  "term_id": "GO:0005886",
  "term_label": "plasma membrane",
  "gene_name": "Olfactory receptor 2T2"
}